hygromycin-B 7''-O-phosphotransferase activity [GO:0008904] (molecular function) Sources: EC:2.7.1.119, RHEA:23388 Relationships: is a type of aminoglycoside phosphotransferase activity [GO:0034071] Definition: Catalysis of the reaction: ATP + hygromycin B = 7''-O-phosphohygromycin B + ADP + 2 H+. Also known as: hygromycin B kinase activity, hygromycin B phosphotransferase activity, hygromycin-B kinase activity, destomic acid ring 7''-O-phosphotransferase activity, APH(7'') activity, ATP:hygromycin-B 7''-O-phosphotransferase activity